{
  "term_label": "spliceosomal complex assembly",
  "gene_name": "Splicing factor 3B subunit 1",
  "gene": "UniProtKB:O75533",
  "gene_symbol": "SF3B1",
  "term_id": "GO:0000245"
}